{
  "gene_symbol": "B3GALT9",
  "gene_name": "Beta-1,3-galactosyltransferase 9",
  "gene": "UniProtKB:A8MXE2",
  "term_id": "GO:0016757",
  "term_label": "glycosyltransferase activity"
}